{
  "term_label": "Unknown molecular function",
  "term_id": "UNKNOWN:0001",
  "gene": "UniProtKB:Q96NR7",
  "gene_symbol": "WWC2-AS2",
  "gene_name": "Putative uncharacterized protein WWC2-AS2"
}